musculoskeletal movement [GO:0050881] (biological process) Definition: The movement of an organism or part of an organism using mechanoreceptors, the nervous system, striated muscle and/or the skeletal system. Relationships: is a type of multicellular organismal movement [GO:0050879]; is a type of GO:0050905 Sources: GOC:dph Subtypes: GO:0050882, GO:0050883